{
  "gene_symbol": "INSYN2B",
  "gene": "UniProtKB:A6NMK8",
  "term_id": "UNKNOWN:0003",
  "gene_name": "Protein INSYN2B",
  "term_label": "Unknown cellular component"
}